lytic exotransglycosylase activity [GO:0140100] (molecular function) Also known as: murein lytic endotransglycosylase E activity Relationships: is a type of peptidoglycan lytic transglycosylase activity [GO:0008933] Definition: Catalysis of the exolytic cleavage of the (1->4)-beta-glycosidic linkage between N-acetylmuramic acid (MurNAc) and N-acetylglucosamine (GlcNAc) residues in peptidoglycan, from either the reducing or the non-reducing ends of the peptidoglycan chains, with concomitant formation of a 1,6-anhydrobond in the MurNAc residue. Sources: EC:4.2.2.n1